{
  "gene_symbol": "FADD",
  "gene": "UniProtKB:Q13158",
  "term_id": "GO:0045089",
  "gene_name": "FAS-associated death domain protein",
  "term_label": "positive regulation of innate immune response"
}